{
  "gene_name": "D(1A) dopamine receptor",
  "gene_symbol": "DRD1",
  "term_id": "GO:0004930",
  "term_label": "G protein-coupled receptor activity",
  "gene": "UniProtKB:P21728"
}